{
  "term_label": "extracellular matrix",
  "gene_name": "CCN family member 4",
  "gene_symbol": "CCN4",
  "gene": "UniProtKB:O95388",
  "term_id": "GO:0031012"
}